{
  "term_label": "riboflavin metabolic process",
  "gene_name": "Riboflavin kinase",
  "gene": "UniProtKB:Q969G6",
  "gene_symbol": "RFK",
  "term_id": "GO:0006771"
}